{
  "term_id": "GO:0051015",
  "gene": "UniProtKB:Q14847",
  "term_label": "actin filament binding",
  "gene_name": "LIM and SH3 domain protein 1",
  "gene_symbol": "LASP1"
}